ganglion formation [GO:0061554] (biological process) Also known as: ganglia formation Sources: GOC:dph Definition: The process that gives rise to ganglion. This process pertains to the initial formation of a structure from unspecified parts. Relationships: is a type of anatomical structure formation involved in morphogenesis [GO:0048646]; is part of ganglion morphogenesis [GO:0061552] Subtypes: cranial ganglion formation [GO:0061560]